regulation of growth plate cartilage chondrocyte proliferation [GO:0003420] (biological process) Sources: GOC:ascb_2009, GOC:dph, GOC:tb Subtypes: GO:0061913, GO:0061914 Relationships: is a type of regulation of cell population proliferation [GO:0042127]; regulates GO:0003419 Definition: Any process that modulates the rate, frequency, or extent of the multiplication or reproduction of chondrocytes in a growing endochondral bone, resulting in the expansion of a cell population.